voltage-gated potassium channel activity involved in bundle of His cell action potential repolarization [GO:0086087] (MF) Relationships: is a type of voltage-gated potassium channel activity involved in cardiac muscle cell action potential repolarization [GO:0086008]; is part of membrane repolarization during bundle of His cell action potential [GO:0086050] Sources: GOC:BHF, GOC:mtg_cardiac_conduct_nov11 Definition: Enables the transmembrane transfer of a potassium ion by a voltage-gated channel through the plasma membrane of a bundle of His cell contributing to the repolarization phase of an action potential. A voltage-gated channel is a channel whose open state is dependent on the voltage across the membrane in which it is embedded.